{
  "gene": "UniProtKB:Q9HCM9",
  "term_id": "GO:0061630",
  "gene_symbol": "TRIM39",
  "gene_name": "E3 ubiquitin-protein ligase TRIM39",
  "term_label": "ubiquitin protein ligase activity"
}